{
  "term_label": "extracellular matrix",
  "gene_symbol": "FBN1",
  "term_id": "GO:0031012",
  "gene": "UniProtKB:P35555",
  "gene_name": "Fibrillin-1"
}